{
  "gene_name": "Putative uncharacterized protein encoded by LINC00158",
  "gene": "UniProtKB:P58513",
  "term_label": "Unknown biological process",
  "term_id": "UNKNOWN:0002",
  "gene_symbol": "LINC00158"
}